cardiac muscle myosin thick filament assembly [GO:0071690] (BP) Sources: GOC:mah Definition: The aggregation, arrangement and bonding together of proteins to form the myosin-based thick filaments of myofibrils in cardiac muscle. Relationships: is a type of striated muscle myosin thick filament assembly [GO:0071688]; is part of cardiac myofibril assembly [GO:0055003]